{
  "term_id": "GO:0003682",
  "term_label": "chromatin binding",
  "gene": "UniProtKB:Q7L190",
  "gene_name": "Developmental pluripotency-associated protein 4",
  "gene_symbol": "DPPA4"
}